{
  "term_id": "GO:0006814",
  "gene_symbol": "CATSPER4",
  "gene_name": "Cation channel sperm-associated protein 4",
  "term_label": "sodium ion transport",
  "gene": "UniProtKB:Q7RTX7"
}